dol-P-Man:Man(5)GlcNAc(2)-PP-Dol alpha-1,3-mannosyltransferase activity [GO:0052925] (molecular function) Also known as: dolichyl-P-Man:Man(5)GlcNAc(2)-PP-dolichyl mannosyltransferase activity, man(5)GlcNAc(2)-PP-Dol mannosyltransferase activity Relationships: is a type of GO:0000033; is a type of GlcNAc(2)-PP-Dol mannosyltransferase activity [GO:0120562] Sources: RHEA:29527 Definition: Catalysis of the reaction: an alpha-D-Man-(1->2)-alpha-D-Man-(1->2)-alpha-D-Man-(1->3)-[alpha-D-Man-(1->6)]-beta-D-Man-(1->4)-beta-D-GlcNAc-(1->4)-alpha-D-GlcNAc-diphospho-di-trans,poly-cis-dolichol + a di-trans,poly-cis-dolichyl beta-D-mannosyl phosphate = an alpha-D-Man-(1->2)-alpha-D-Man-(1->2)-alpha-D-Man-(1->3)-[alpha-D-Man-(1->3)-alpha-D-Man-(1->6)]-beta-D-Man-(1->4)-beta-D-GlcNAc-(1->4)-alpha-D-GlcNAc-diphospho-di-trans,poly-cis-dolichol + a di-trans,poly-cis-dolichyl phosphate + H+.